{
  "gene": "UniProtKB:Q8NGP6",
  "gene_name": "Olfactory receptor 5M8",
  "term_label": "G protein-coupled receptor signaling pathway",
  "gene_symbol": "OR5M8",
  "term_id": "GO:0007186"
}